{
  "term_id": "GO:0000981",
  "gene_name": "Zinc finger protein 75A",
  "gene": "UniProtKB:Q96N20",
  "gene_symbol": "ZNF75A",
  "term_label": "DNA-binding transcription factor activity, RNA polymerase II-specific"
}